{
  "term_label": "RNA polymerase II transcription regulatory region sequence-specific DNA binding",
  "term_id": "GO:0000977",
  "gene_name": "Fer3-like protein",
  "gene": "UniProtKB:Q96RJ6",
  "gene_symbol": "FERD3L"
}